{
  "gene": "UniProtKB:P0CG39",
  "gene_symbol": "POTEJ",
  "term_id": "GO:0035267",
  "term_label": "NuA4 histone acetyltransferase complex",
  "gene_name": "POTE ankyrin domain family member J"
}